{
  "term_label": "Unknown molecular function",
  "term_id": "UNKNOWN:0001",
  "gene_name": "Tetraspanin-10",
  "gene": "UniProtKB:Q9H1Z9",
  "gene_symbol": "TSPAN10"
}